cytoskeletal regulatory protein binding [GO:0005519] (molecular function) Definition: Binding to a protein involved in modulating the reorganization of the cytoskeleton. References: PMID:15163540 Sources: GOC:go_curators Relationships: is a type of cytoskeletal protein binding [GO:0008092]